{
  "term_label": "autophagosome assembly",
  "gene": "UniProtKB:Q9H0Y0",
  "term_id": "GO:0000045",
  "gene_symbol": "ATG10",
  "gene_name": "Ubiquitin-like-conjugating enzyme ATG10"
}